NLRP1 inflammasome complex assembly [GO:1904784] (BP) Note: The aggregation, arrangement and bonding together of a set of components to form the NLRP1 inflammasome complex, occurring at the level of an individual cell. Definition: The aggregation, arrangement and bonding together of a set of components to form a NLRP1 inflammasome complex. Relationships: is a type of canonical inflammasome complex assembly [GO:0140632] Also known as: NALP1 inflammasome complex assembly, NALP1 inflammasome complex formation, NLRP1 inflammasome complex formation References: PMID:19124602 Sources: GOC:TermGenie, GO_REF:0000079